{
  "term_id": "GO:0004674",
  "gene_name": "Serine_threonine-protein kinase MAK",
  "gene_symbol": "MAK",
  "term_label": "protein serine/threonine kinase activity",
  "gene": "UniProtKB:P20794"
}